{
  "gene_symbol": "SOX6",
  "term_label": "regulation of transcription by RNA polymerase II",
  "term_id": "GO:0006357",
  "gene": "UniProtKB:P35712",
  "gene_name": "Transcription factor SOX-6"
}